{
  "term_label": "Unknown biological process",
  "gene_name": "Uncharacterized protein IDI2-AS1",
  "gene": "UniProtKB:Q9NZ38",
  "gene_symbol": "IDI2-AS1",
  "term_id": "UNKNOWN:0002"
}